{
  "term_label": "Unknown molecular function",
  "gene_name": "Putative methyltransferase NSUN5C",
  "term_id": "UNKNOWN:0001",
  "gene": "UniProtKB:Q63ZY6",
  "gene_symbol": "NSUN5P2"
}